{
  "term_label": "condensin complex",
  "term_id": "GO:0000796",
  "gene_name": "Condensin complex subunit 2",
  "gene": "UniProtKB:Q15003",
  "gene_symbol": "NCAPH"
}